{
  "term_id": "GO:0043171",
  "gene": "UniProtKB:A6NEC2",
  "gene_name": "Puromycin-sensitive aminopeptidase-like protein",
  "gene_symbol": "NPEPPSL1",
  "term_label": "peptide catabolic process"
}